{
  "term_label": "diphosphoinositol polyphosphate metabolic process",
  "gene_symbol": "NUDT10",
  "term_id": "GO:0071543",
  "gene": "UniProtKB:Q8NFP7",
  "gene_name": "Diphosphoinositol polyphosphate phosphohydrolase 3-alpha"
}